{
  "gene_symbol": "PPP3CC",
  "term_id": "GO:0005516",
  "gene_name": "Serine_threonine-protein phosphatase 2B catalytic subunit gamma isoform",
  "term_label": "calmodulin binding",
  "gene": "UniProtKB:P48454"
}